{
  "gene": "UniProtKB:Q8N1T3",
  "term_label": "microfilament motor activity",
  "gene_symbol": "MYO1H",
  "gene_name": "Unconventional myosin-Ih",
  "term_id": "GO:0000146"
}